neutral sphingomyelin phosphodiesterase activity [GO:0061751] (molecular function) Definition: Catalysis of the reaction: H2O + sphingomyelin = ceramide + choline phosphate + H+ in a neutral environment. References: PMID:26493087 Sources: GOC:dph Also known as: neutral SMase, neutral sphingomyelinase Relationships: is a type of sphingomyelin phosphodiesterase activity [GO:0004767]